{
  "term_label": "Unknown molecular function",
  "gene": "UniProtKB:Q9HBH5",
  "gene_symbol": "RDH14",
  "term_id": "UNKNOWN:0001",
  "gene_name": "Retinol dehydrogenase 14"
}